{
  "term_id": "GO:0001669",
  "gene_symbol": "SPACA9",
  "term_label": "acrosomal vesicle",
  "gene_name": "Sperm acrosome-associated protein 9",
  "gene": "UniProtKB:Q96E40"
}